basophil homeostasis [GO:1990960] (biological process) Relationships: is a type of GO:0001776; is a type of GO:0002262 Also known as: basophilic leucocyte homeostasis References: PMID:10606160 Definition: The process of regulating the proliferation and elimination of basophils such that the total number of basophils within a whole or part of an organism is stable over time in the absence of an outside stimulus.